{
  "gene": "UniProtKB:Q96CG8",
  "term_label": "prostaglandin-endoperoxide synthase activity",
  "gene_name": "Collagen triple helix repeat-containing protein 1",
  "gene_symbol": "CTHRC1",
  "term_id": "GO:0004666"
}